cell motility in response to potassium ion [GO:0097230] (biological process) References: PMID:19363786, PMID:21239624 Sources: GOC:pf Relationships: is_a cell motility [GO:0048870]; is part of GO:0035865 Also known as: K+ facilitation of cell motility, potassium ion facilitation of cell motility Definition: Any process involved in the controlled self-propelled movement of a cell that results in translocation of the cell from one place to another as a result of a potassium ion stimulus.